{
  "gene_name": "Eukaryotic translation elongation factor 1 epsilon-1",
  "term_label": "aminoacyl-tRNA synthetase multienzyme complex",
  "gene_symbol": "EEF1E1",
  "term_id": "GO:0017101",
  "gene": "UniProtKB:O43324"
}